protein export from nucleus [GO:0006611] (biological process) Regulation: regulated by regulation of protein export from nucleus [GO:0046825]; negatively regulated by negative regulation of protein export from nucleus [GO:0046826]; positively regulated by positive regulation of protein export from nucleus [GO:0046827] Sources: GOC:jl Definition: The directed movement of a protein from the nucleus into the cytoplasm. Also known as: protein export from cell nucleus, protein export out of nucleus, protein transport from nucleus to cytoplasm, protein-nucleus export, copper-induced protein export from nucleus Relationships: is a type of intracellular protein transport [GO:0006886]; is a type of nuclear export [GO:0051168]